monoatomic cation transmembrane transporter activity [GO:0008324] (molecular function) Relationships: is a type of monoatomic ion transmembrane transporter activity [GO:0015075]; is part of monoatomic cation transmembrane transport [GO:0098655] Definition: Enables the transfer of cation from one side of a membrane to the other. Subtypes: monoatomic cation channel activity [GO:0005261], GO:0015078, solute:monoatomic cation symporter activity [GO:0015294], ATPase-coupled monoatomic cation transmembrane transporter activity [GO:0019829], silicon efflux transmembrane transporter activity [GO:0032523], GO:0046583, GO:0046873, amino acid:monoatomic cation antiporter activity [GO:0140848] Sources: GOC:dgf, GOC:mtg_transport, ISBN:0815340729 Also known as: cation transmembrane transporter activity, transmembrane cation transporter activity